{
  "gene_name": "Transcription regulator protein BACH2",
  "term_id": "GO:0000978",
  "gene": "UniProtKB:Q9BYV9",
  "term_label": "RNA polymerase II cis-regulatory region sequence-specific DNA binding",
  "gene_symbol": "BACH2"
}